phospholipase B activity [GO:0102545] (molecular function) Definition: Catalysis of the reaction: a 1,2-diacyl-sn-glycero-3-phosphocholine + 2 H2O = sn-glycerol 3-phosphocholine + 2 a carboxylate + 2 H+. Sources: RHEA:32907 Also known as: phosphatidyl phospholipase B activity Relationships: is a type of GO:0004620